{
  "term_id": "GO:0055038",
  "gene_symbol": "RAB11FIP4",
  "gene": "UniProtKB:Q86YS3",
  "gene_name": "Rab11 family-interacting protein 4",
  "term_label": "recycling endosome membrane"
}